{
  "gene_name": "Glycogenin-1",
  "gene": "UniProtKB:P46976",
  "term_label": "glycogen biosynthetic process",
  "term_id": "GO:0005978",
  "gene_symbol": "GYG1"
}